3',5'-nucleotide bisphosphate phosphatase activity [GO:0097657] (molecular function) Definition: Catalysis of the reaction: 3',5'-nucleoside bisphosphate + H20 = 5'-nucleoside monophosphate + phosphate. References: PMID:24401123 Sources: GOC:jh2, RHEA:43532 Relationships: is a type of phosphatase activity [GO:0016791]